{
  "gene_symbol": "GABRR1",
  "term_label": "chloride transmembrane transport",
  "gene": "UniProtKB:P24046",
  "gene_name": "Gamma-aminobutyric acid receptor subunit rho-1",
  "term_id": "GO:1902476"
}